positive regulation of oogenesis [GO:1905881] (biological process) Relationships: is a type of positive regulation of cell development [GO:0010720]; is a type of GO:0051240; is a type of regulation of oogenesis [GO:1905879]; is a type of GO:2000243; positively regulates oogenesis [GO:0048477] Definition: Any process that activates or increases the frequency, rate or extent of oogenesis. References: PMID:26434723 Sources: GOC:TermGenie, GO_REF:0000058 Also known as: positive regulation of ovum development, up regulation of oogenesis, up regulation of ovum development, up-regulation of oogenesis, up-regulation of ovum development, upregulation of oogenesis, upregulation of ovum development, activation of oogenesis, activation of ovum development